negative regulation of hepatic stellate cell contraction [GO:0061875] (biological process) Relationships: is a type of negative regulation of cellular process [GO:0048523]; is a type of regulation of hepatic stellate cell contraction [GO:0061873]; negatively regulates hepatic stellate cell contraction [GO:0061872] Definition: Any process that modulates stops, prevents, or reduces the frequency, rate or extent of hepatic stellate cell contraction. References: PMID:24204762